{
  "gene_name": "Protein S100-A8",
  "gene": "UniProtKB:P05109",
  "gene_symbol": "S100A8",
  "term_label": "cytoplasm",
  "term_id": "GO:0005737"
}